{
  "term_id": "GO:0005634",
  "term_label": "nucleus",
  "gene": "UniProtKB:P51608",
  "gene_name": "Methyl-CpG-binding protein 2",
  "gene_symbol": "MECP2"
}